{
  "gene": "UniProtKB:P10768",
  "gene_symbol": "ESD",
  "term_label": "cytosol",
  "term_id": "GO:0005829",
  "gene_name": "S-formylglutathione hydrolase"
}